lactate-malate transhydrogenase activity [GO:0050042] (molecular function) Sources: EC:1.1.99.7, RHEA:10984 Also known as: (S)-lactate:oxaloacetate oxidoreductase activity, malate-lactate transhydrogenase activity Definition: Catalysis of the reaction: (S)-lactate + oxaloacetate = malate + pyruvate. Relationships: is_a GO:0016614